{
  "gene": "UniProtKB:Q13316",
  "gene_symbol": "DMP1",
  "gene_name": "Dentin matrix acidic phosphoprotein 1",
  "term_id": "GO:0031012",
  "term_label": "extracellular matrix"
}